{
  "term_label": "cytoplasm",
  "term_id": "GO:0005737",
  "gene_name": "C-Jun-amino-terminal kinase-interacting protein 1",
  "gene_symbol": "MAPK8IP1",
  "gene": "UniProtKB:Q9UQF2"
}